{
  "gene": "UniProtKB:O15375",
  "term_id": "GO:0016323",
  "gene_name": "Monocarboxylate transporter 6",
  "gene_symbol": "SLC16A5",
  "term_label": "basolateral plasma membrane"
}